{
  "gene_name": "Serine_threonine-protein kinase Nek11",
  "gene": "UniProtKB:Q8NG66",
  "term_id": "GO:0031573",
  "term_label": "mitotic intra-S DNA damage checkpoint signaling",
  "gene_symbol": "NEK11"
}